regulation of dendrite extension [GO:1903859] (biological process) Definition: Any process that modulates the frequency, rate or extent of dendrite extension. References: PMID:24898855 Sources: GOC:PARL, GOC:TermGenie, GOC:pad, GO_REF:0000058 Note: An example of this is Mul1 in mouse (UniProt ID Q8VCM5) in PMID:24898855 inferred from mutant phenotype. Relationships: is a type of GO:0001558; is a type of regulation of cell morphogenesis [GO:0022604]; is a type of regulation of developmental growth [GO:0048638]; RO_0002211 dendrite extension [GO:0097484] Subtypes: negative regulation of dendrite extension [GO:1903860], positive regulation of dendrite extension [GO:1903861]